{
  "term_label": "extracellular space",
  "term_id": "GO:0005615",
  "gene_name": "Secreted frizzled-related protein 2",
  "gene": "UniProtKB:Q96HF1",
  "gene_symbol": "SFRP2"
}